actin-based cell projection [GO:0098858] (cellular component) Relationships: is a type of plasma membrane bounded cell projection [GO:0120025]; has part actin filament [GO:0005884] Subtypes: GO:0005902, filopodium [GO:0030175], stereocilium [GO:0032420], cytospinule [GO:0160231] Definition: A cell projection supported by an assembly of actin filaments, and which lacks microtubules. References: PMID:15661519